{
  "term_id": "GO:0000981",
  "gene": "UniProtKB:Q9BYN7",
  "gene_name": "Zinc finger protein 341",
  "gene_symbol": "ZNF341",
  "term_label": "DNA-binding transcription factor activity, RNA polymerase II-specific"
}